acylphosphatase activity [GO:0003998] (molecular function) Sources: EC:3.6.1.7 Definition: Catalysis of the reaction: an acyl phosphate + H2O = a carboxylate + phosphate. Relationships: is a type of pyrophosphatase activity [GO:0016462] Also known as: 1,3-diphosphoglycerate phosphatase activity, GP 1-3, Ho 1-3, acetic phosphatase activity, acetylphosphatase activity, acylphosphate phosphohydrolase activity